phosphatidylinositol binding [GO:0035091] (molecular function) Definition: Binding to an inositol-containing glycerophospholipid, i.e. phosphatidylinositol (PtdIns) and its phosphorylated derivatives. References: PMID:11395417 Sources: GOC:bf, ISBN:0198506732 Subtypes: 1-phosphatidylinositol binding [GO:0005545], GPI anchor binding [GO:0034235], phosphatidylinositol phosphate binding [GO:1901981] Relationships: is a type of GO:0005543 Also known as: phosphoinositide binding